{
  "gene_name": "NACHT, LRR and PYD domains-containing protein 1",
  "gene_symbol": "NLRP1",
  "gene": "UniProtKB:Q9C000",
  "term_id": "GO:0072559",
  "term_label": "NLRP3 inflammasome complex"
}